spermine oxidase (propane-1,3-diamine-forming) activity [GO:0052900] (molecular function) Relationships: is a type of polyamine oxidase activity [GO:0046592] Also known as: polyamine oxidase (propane-1,3-diamine-forming) activity Definition: Catalysis of the reaction: H2O + O2 + spermine = 1,3-diaminopropane + H2O2 + N-(3-aminopropyl)-4-aminobutanal. Weak activity on N(1)-acetylspermine and spermine. Sources: EC:1.5.3.14, RHEA:25824